{
  "gene_symbol": "B3GALT4",
  "term_id": "GO:0016757",
  "term_label": "glycosyltransferase activity",
  "gene": "UniProtKB:O96024",
  "gene_name": "Beta-1,3-galactosyltransferase 4"
}